{
  "term_id": "GO:0051131",
  "gene": "UniProtKB:Q8TAM1",
  "term_label": "chaperone-mediated protein complex assembly",
  "gene_symbol": "BBS10",
  "gene_name": "Bardet-Biedl syndrome 10 protein"
}